{
  "gene_name": "Cyclin-dependent kinase 3",
  "term_label": "cytoplasm",
  "gene": "UniProtKB:Q00526",
  "term_id": "GO:0005737",
  "gene_symbol": "CDK3"
}